trichloroethylene metabolic process [GO:0018979] (biological process) Sources: GOC:jl Relationships: is a type of halogenated hydrocarbon metabolic process [GO:0042197] Subtypes: trichloroethylene catabolic process [GO:0050696] Also known as: TCE metabolic process, TCE metabolism, trichloroethene metabolic process, trichloroethene metabolism, trichloroethylene metabolism Definition: The chemical reactions and pathways involving trichloroethylene, a toxic, colorless, photoreactive, chlorinated hydrocarbon liquid, commonly used as a metal degreaser and solvent.